cardiac myofibril [GO:0097512] (cellular component) Definition: A cardiac myofibril is a myofibril specific to cardiac muscle cells. Relationships: is a type of GO:0030016 Sources: GOC:cjm, GOC:devbiol